{
  "gene": "UniProtKB:Q96J01",
  "term_label": "mRNA export from nucleus",
  "gene_symbol": "THOC3",
  "gene_name": "THO complex subunit 3",
  "term_id": "GO:0006406"
}